{
  "gene_symbol": "LRRC20",
  "term_id": "UNKNOWN:0002",
  "gene": "UniProtKB:Q8TCA0",
  "term_label": "Unknown biological process",
  "gene_name": "Leucine-rich repeat-containing protein 20"
}